leukocyte proliferation [GO:0070661] (BP) Subtypes: osteoclast proliferation [GO:0002158], mononuclear cell proliferation [GO:0032943], monocyte proliferation [GO:0061516], GO:0061517, mast cell proliferation [GO:0070662] Relationships: is a type of cell population proliferation [GO:0008283] Definition: The expansion of a leukocyte population by cell division. Regulation: regulated by regulation of leukocyte proliferation [GO:0070663]; negatively regulated by GO:0070664; positively regulated by GO:0070665 Sources: GOC:add